isoliquiritigenin 2'-O-methyltransferase activity [GO:0033802] (molecular function) Relationships: is a type of GO:0008171; is a type of GO:0008757 Definition: Catalysis of the reaction: S-adenosyl-L-methionine + isoliquiritigenin = 2'-O-methylisoliquiritigenin + S-adenosyl-L-homocysteine + H+. Also known as: CHMT, S-adenosyl-L-methionine:isoliquiritigenin 2'-O-methyltransferase activity, chalcone OMT Sources: EC:2.1.1.154, RHEA:21608